L-idonate 5-dehydrogenase [NAD(P)+] activity [GO:0050572] (MF) Subtypes: GO:0102198 Also known as: L-idonate:NAD(P)+ oxidoreductase activity Definition: Catalysis of the reaction: L-idonate + NAD(P)+ = 5-dehydrogluconate + NAD(P)H + H+. Relationships: is a type of oxidoreductase activity, acting on the CH-OH group of donors, NAD or NADP as acceptor [GO:0016616] Sources: EC:1.1.1.264